SNARE complex disassembly [GO:0035494] (biological process) Relationships: is a type of GO:0032984; is part of vesicle-mediated transport [GO:0016192] References: PMID:11697877 Sources: GOC:rb Regulation: regulated by GO:0035495; positively regulated by positive regulation of SNARE complex disassembly [GO:0035540]; negatively regulated by GO:0035541 Definition: The disaggregation of the SNARE protein complex into its constituent components. The SNARE complex is a protein complex involved in membrane fusion; a stable ternary complex consisting of a four-helix bundle, usually formed from one R-SNARE and three Q-SNAREs with an ionic layer sandwiched between hydrophobic layers.